{
  "term_label": "intraciliary transport involved in cilium assembly",
  "gene_symbol": "IFT74",
  "gene_name": "Intraflagellar transport protein 74 homolog",
  "gene": "UniProtKB:Q96LB3",
  "term_id": "GO:0035735"
}